{
  "term_id": "GO:0048870",
  "gene": "UniProtKB:Q6S8J3",
  "gene_name": "POTE ankyrin domain family member E",
  "term_label": "cell motility",
  "gene_symbol": "POTEE"
}